{
  "gene": "UniProtKB:P55318",
  "term_id": "UNKNOWN:0003",
  "gene_symbol": "FOXA3",
  "term_label": "Unknown cellular component",
  "gene_name": "Hepatocyte nuclear factor 3-gamma"
}